{
  "term_label": "barbed-end actin filament capping",
  "gene_symbol": "TWF1",
  "gene_name": "Twinfilin-1",
  "term_id": "GO:0051016",
  "gene": "UniProtKB:Q12792"
}